symbiont-containing vacuole [GO:0020003] (cellular component) Sources: GOC:jl, GOC:mb Relationships: is a type of cellular anatomical structure [GO:0110165] Definition: Membrane-bounded vacuole within a host cell in which a symbiont organism resides. The vacuole membrane is derived from both the host and symbiont. Note: Note that this term does not have a relationship to 'vacuole ; GO:0005773' because it does not fit the definition of a vacuole; the parasitophorous vacuole was so named because it resembles a vacuole in the microscope. Also known as: SCV, parasitophorous vacuole, Salmonella-containing vacuole, bacterium-containing vacuole, pathogen-occupied vacuole